negative regulation of epidermal cell differentiation [GO:0045605] (biological process) Sources: GOC:go_curators Subtypes: negative regulation of inner ear auditory receptor cell differentiation [GO:0045608], negative regulation of keratinocyte differentiation [GO:0045617] Also known as: down regulation of epidermal cell differentiation, down-regulation of epidermal cell differentiation, downregulation of epidermal cell differentiation, inhibition of epidermal cell differentiation, negative regulation of hypodermal cell differentiation Relationships: is a type of GO:0030857; is_a regulation of epidermal cell differentiation [GO:0045604]; is_a GO:0045683; negatively regulates epidermal cell differentiation [GO:0009913] Definition: Any process that stops, prevents, or reduces the frequency, rate or extent of epidermal cell differentiation.